{
  "gene_name": "CCAAT_enhancer-binding protein epsilon",
  "gene": "UniProtKB:Q15744",
  "term_label": "DNA-binding transcription factor activity, RNA polymerase II-specific",
  "term_id": "GO:0000981",
  "gene_symbol": "CEBPE"
}